{
  "term_id": "GO:0003724",
  "gene": "UniProtKB:Q9NR30",
  "term_label": "RNA helicase activity",
  "gene_name": "Nucleolar RNA helicase 2",
  "gene_symbol": "DDX21"
}